{
  "term_id": "GO:0005634",
  "gene": "UniProtKB:P28356",
  "gene_name": "Homeobox protein Hox-D9",
  "gene_symbol": "HOXD9",
  "term_label": "nucleus"
}